{
  "gene": "UniProtKB:Q15427",
  "term_label": "precatalytic spliceosome",
  "gene_name": "Splicing factor 3B subunit 4",
  "term_id": "GO:0071011",
  "gene_symbol": "SF3B4"
}